metanephric renal vesicle morphogenesis [GO:0072283] (biological process) Definition: The process in which the anatomical structures of the metanephric renal vesicle are generated and organized. The renal vesicle is the primordial structure of the metanephric nephron epithelium, and is formed by the condensation of mesenchymal cells. Sources: GOC:mtg_kidney_jan10 Relationships: is a type of GO:0072077; is part of metanephric nephron morphogenesis [GO:0072273]